{
  "term_id": "GO:0004864",
  "gene_symbol": "ARPP19",
  "gene": "UniProtKB:P56211",
  "term_label": "protein phosphatase inhibitor activity",
  "gene_name": "cAMP-regulated phosphoprotein 19"
}